nematode male tail tip morphogenesis [GO:0045138] (biological process) References: PMID:16806150, PMID:18050419, PMID:21408209, PMID:7409314 Sources: GOC:kmv Regulation: regulated by regulation of nematode male tail tip morphogenesis [GO:0110037]; negatively regulated by negative regulation of nematode male tail tip morphogenesis [GO:0110038]; positively regulated by GO:0110039 Definition: The process in which the anatomical structure of the adult male tail tip is generated and organized. In some species of rhabitid nematodes, the male tail tip undergoes a morphological change such that the most posterior hypodermal cells in the tail (hyp8-11 in C. elegans) fuse and retract anteriorly, changing the shape of the tail from a pointed, tapered cone, or spike, to a rounded, blunt dome. Also known as: male tail morphogenesis, male tail tip morphogenesis, tail tip morphogenesis Relationships: is a type of male anatomical structure morphogenesis [GO:0090598]